{
  "gene": "UniProtKB:P01236",
  "term_id": "GO:0007166",
  "term_label": "cell surface receptor signaling pathway",
  "gene_symbol": "PRL",
  "gene_name": "Prolactin"
}